{
  "term_id": "GO:0005737",
  "gene_name": "Ubiquitin-associated and SH3 domain-containing protein B",
  "term_label": "cytoplasm",
  "gene": "UniProtKB:Q8TF42",
  "gene_symbol": "UBASH3B"
}